{
  "gene": "UniProtKB:Q3SYB3",
  "gene_symbol": "FOXD4L6",
  "term_id": "GO:0000981",
  "term_label": "DNA-binding transcription factor activity, RNA polymerase II-specific",
  "gene_name": "Forkhead box protein D4-like 6"
}